{
  "gene_name": "Uncharacterized protein",
  "term_id": "UNKNOWN:0003",
  "gene_symbol": "LOC647264",
  "gene": "UniProtKB:A0A3B3IRS2",
  "term_label": "Unknown cellular component"
}